{
  "term_id": "UNKNOWN:0003",
  "gene_symbol": "DNM1P46",
  "term_label": "Unknown cellular component",
  "gene_name": "Putative GED domain-containing protein DNM1P46",
  "gene": "UniProtKB:Q6ZS02"
}